{
  "gene": "UniProtKB:Q5T5A4",
  "gene_symbol": "CFAP276",
  "term_id": "UNKNOWN:0002",
  "term_label": "Unknown biological process",
  "gene_name": "Cilia- and flagella-associated protein 276"
}